{
  "term_id": "GO:0098978",
  "term_label": "glutamatergic synapse",
  "gene_symbol": "EFNB3",
  "gene": "UniProtKB:Q15768",
  "gene_name": "Ephrin-B3"
}